spindle pole [GO:0000922] (cellular component) Definition: Either of the ends of a spindle, where spindle microtubules are organized; usually contains a microtubule organizing center and accessory molecules, spindle microtubules and astral microtubules. Subtypes: GO:0090619, mitotic spindle pole [GO:0097431] Sources: GOC:clt Relationships: is a type of cellular anatomical structure [GO:0110165]; is part of GO:0005819